{
  "gene": "UniProtKB:Q16778",
  "gene_symbol": "H2BC21",
  "term_id": "GO:0003677",
  "term_label": "DNA binding",
  "gene_name": "Histone H2B type 2-E"
}